{
  "gene": "UniProtKB:P28907",
  "gene_symbol": "CD38",
  "term_label": "positive regulation of B cell proliferation",
  "gene_name": "ADP-ribosyl cyclase_cyclic ADP-ribose hydrolase 1",
  "term_id": "GO:0030890"
}